{
  "term_id": "GO:0000978",
  "gene": "UniProtKB:P15622",
  "term_label": "RNA polymerase II cis-regulatory region sequence-specific DNA binding",
  "gene_name": "Zinc finger protein 250",
  "gene_symbol": "ZNF250"
}